{
  "gene_symbol": "ACVR1C",
  "term_label": "activin receptor complex",
  "term_id": "GO:0048179",
  "gene_name": "Activin receptor type-1C",
  "gene": "UniProtKB:Q8NER5"
}